{
  "term_id": "UNKNOWN:0001",
  "gene_symbol": "WSCD2",
  "term_label": "Unknown molecular function",
  "gene": "UniProtKB:Q2TBF2",
  "gene_name": "Sialate:O-sulfotransferase 2"
}